{
  "gene_name": "Protein scribble homolog",
  "gene": "UniProtKB:Q14160",
  "gene_symbol": "SCRIB",
  "term_id": "GO:0045211",
  "term_label": "postsynaptic membrane"
}